{
  "term_label": "GTPase activator activity",
  "gene_name": "TBC1 domain family member 16",
  "gene_symbol": "TBC1D16",
  "term_id": "GO:0005096",
  "gene": "UniProtKB:Q8TBP0"
}